isopentenyl diphosphate metabolic process [GO:0046490] (biological process) Relationships: is a type of GO:0006644 Also known as: IPP metabolic process, IPP metabolism, isopentenyl diphosphate metabolism, isopentenyl pyrophosphate metabolic process, isopentenyl pyrophosphate metabolism Subtypes: isopentenyl diphosphate biosynthetic process [GO:0009240] Definition: The chemical reactions and pathways involving isopentenyl diphosphate, an isomer of dimethylallyl diphosphate and the key precursor of all isoprenoids. Sources: ISBN:0198506732